{
  "gene_symbol": "C20orf173",
  "gene": "UniProtKB:Q96LM9",
  "term_label": "beta-galactoside (CMP) alpha-2,3-sialyltransferase activity",
  "term_id": "GO:0003836",
  "gene_name": "Uncharacterized protein C20orf173"
}